{
  "term_label": "microtubule organizing center",
  "gene": "UniProtKB:Q15691",
  "term_id": "GO:0005815",
  "gene_name": "Microtubule-associated protein RP_EB family member 1",
  "gene_symbol": "MAPRE1"
}